{
  "gene_name": "Integral membrane protein 2A",
  "gene": "UniProtKB:O43736",
  "term_id": "GO:0005794",
  "term_label": "Golgi apparatus",
  "gene_symbol": "ITM2A"
}